{
  "gene_name": "Zinc finger protein 429",
  "gene": "UniProtKB:Q86V71",
  "term_id": "GO:0005634",
  "gene_symbol": "ZNF429",
  "term_label": "nucleus"
}